{
  "term_id": "GO:0046513",
  "term_label": "ceramide biosynthetic process",
  "gene": "UniProtKB:Q8NFR3",
  "gene_name": "Serine palmitoyltransferase small subunit B",
  "gene_symbol": "SPTSSB"
}